negative regulation of activated T cell autonomous cell death [GO:0070240] (biological process) Also known as: negative regulation of ACAD, negative regulation of activated T cell apoptosis, negative regulation of activated cell autonomous cell death, down regulation of activated T cell autonomous cell death, down-regulation of activated T cell autonomous cell death, downregulation of activated T cell autonomous cell death, negative regulation of activated T lymphocyte autonomous cell death, negative regulation of activated T-cell autonomous cell death, negative regulation of activated T-lymphocyte autonomous cell death, inhibition of activated T cell autonomous cell death Sources: GOC:add, GOC:mtg_apoptosis, ISBN:0781765196 Relationships: is a type of negative regulation of immune system process [GO:0002683]; is a type of GO:0070233; is a type of regulation of activated T cell autonomous cell death [GO:0070239]; negatively regulates activated T cell autonomous cell death [GO:0070238] Definition: Any process that stops, prevents, or reduces the frequency, rate or extent of activated T cell autonomous cell death.